{
  "gene_name": "High mobility group protein HMG-I_HMG-Y",
  "term_id": "GO:0035556",
  "term_label": "intracellular signal transduction",
  "gene": "UniProtKB:P17096",
  "gene_symbol": "HMGA1"
}